{
  "gene_name": "Lanosterol synthase",
  "gene": "UniProtKB:P48449",
  "term_id": "GO:0000250",
  "gene_symbol": "LSS",
  "term_label": "lanosterol synthase activity"
}